{
  "gene_name": "Caveolin-2",
  "term_label": "cell differentiation",
  "gene": "UniProtKB:P51636",
  "term_id": "GO:0030154",
  "gene_symbol": "CAV2"
}